{
  "gene": "UniProtKB:Q6P2D0",
  "gene_name": "Zinc finger protein 1 homolog",
  "term_label": "nucleus",
  "term_id": "GO:0005634",
  "gene_symbol": "ZFP1"
}